oxidoreductase activity, acting on a sulfur group of donors, NAD(P) as acceptor [GO:0016668] (molecular function) Sources: GOC:jl Subtypes: dihydrolipoyl dehydrogenase (NADH) activity [GO:0004148], glutathione-disulfide reductase (NADPH) activity [GO:0004362], GO:0004783, alkyl hydroperoxide reductase activity [GO:0008785], GO:0015042, dissimilatory sulfite reductase (NADH) activity [GO:0018551], GO:0047134, bis-gamma-L-glutamylcystine reductase (NADPH) activity [GO:0047135], GO:0050445, CoA-disulfide reductase (NADPH) activity [GO:0050451], CoA-glutathione reductase (NADPH) activity [GO:0050452], L-cystine reductase (NADH) activity [GO:0050456], GO:0050627, 2-oxopropyl-CoM reductase (carboxylating) activity [GO:0050628], GO:0098622 Also known as: oxidoreductase activity, acting on NADH or NADPH, disulfide as acceptor, oxidoreductase activity, acting on NADH or NADPH, disulphide as acceptor, oxidoreductase activity, acting on sulphur group of donors, NAD or NADP as acceptor, oxidoreductase activity, acting on a sulfur group of donors, NAD or NADP as acceptor Definition: Catalysis of an oxidation-reduction (redox) reaction in which a sulfur-containing group acts as a hydrogen or electron donor and reduces NAD or NADP. Relationships: is a type of GO:0016667